{
  "gene_name": "RNA-binding protein 20",
  "term_label": "nucleus",
  "gene_symbol": "RBM20",
  "gene": "UniProtKB:Q5T481",
  "term_id": "GO:0005634"
}